{
  "gene_name": "PDZ domain-containing protein 7",
  "term_id": "GO:0005886",
  "term_label": "plasma membrane",
  "gene_symbol": "PDZD7",
  "gene": "UniProtKB:Q9H5P4"
}